{
  "gene_name": "Blood group Rh(CE) polypeptide",
  "term_id": "GO:0005886",
  "term_label": "plasma membrane",
  "gene_symbol": "RHCE",
  "gene": "UniProtKB:P18577"
}